{
  "gene_name": "3-hydroxyanthranilate 3,4-dioxygenase",
  "term_id": "GO:0046874",
  "gene": "UniProtKB:P46952",
  "gene_symbol": "HAAO",
  "term_label": "quinolinate metabolic process"
}